{
  "gene": "UniProtKB:P48230",
  "gene_symbol": "TM4SF4",
  "term_id": "UNKNOWN:0002",
  "gene_name": "Transmembrane 4 L6 family member 4",
  "term_label": "Unknown biological process"
}